{
  "gene": "UniProtKB:A6NEQ0",
  "gene_name": "RNA-binding motif protein, Y chromosome, family 1 member E",
  "term_id": "GO:0003729",
  "gene_symbol": "RBMY1E",
  "term_label": "mRNA binding"
}